{
  "gene_name": "Intermembrane lipid transfer protein VPS13D",
  "term_id": "GO:0007005",
  "gene": "UniProtKB:Q5THJ4",
  "gene_symbol": "VPS13D",
  "term_label": "mitochondrion organization"
}